{
  "gene_symbol": "ARMC7",
  "term_label": "Unknown molecular function",
  "term_id": "UNKNOWN:0001",
  "gene": "UniProtKB:Q9H6L4",
  "gene_name": "Armadillo repeat-containing protein 7"
}